adenylyl-sulfate reductase (thioredoxin) activity [GO:0043866] (molecular function) Definition: Catalysis of the reaction: AMP + sulfite + thioredoxin disulfide = 5'-adenylyl sulfate + thioredoxin. Sources: EC:1.8.4.10 Also known as: AMP, sulfite:thioredoxin-disulfide oxidoreductase (adenosine-5'-phosphosulfate-forming), thioredoxin-dependent 5'-adenylylsulfate reductase activity, AMP,sulfite:thioredoxin-disulfide oxidoreductase (adenosine-5'-phosphosulfate-forming) Relationships: is_a oxidoreductase activity, acting on a sulfur group of donors, disulfide as acceptor [GO:0016671]